{
  "term_label": "Unknown biological process",
  "gene_name": "CXXC-type zinc finger protein 5",
  "term_id": "UNKNOWN:0002",
  "gene": "UniProtKB:Q7LFL8",
  "gene_symbol": "CXXC5"
}